{
  "term_label": "structural molecule activity",
  "gene": "UniProtKB:Q9UPN3",
  "gene_name": "Microtubule-actin cross-linking factor 1, isoforms 1_2_3_4_5",
  "gene_symbol": "MACF1",
  "term_id": "GO:0005198"
}